{
  "term_id": "GO:0005886",
  "term_label": "plasma membrane",
  "gene_symbol": "LAMP1",
  "gene_name": "Lysosome-associated membrane glycoprotein 1",
  "gene": "UniProtKB:P11279"
}